MutLbeta complex [GO:0032390] (cellular component) Relationships: is a type of mismatch repair complex [GO:0032300]; is_a nuclear protein-containing complex [GO:0140513] Definition: A heterodimer involved in the recognition of base-base and small insertion/deletion mismatches. In human the complex consists of two subunits, MLH1 and PMS1. Also known as: MMR complex, MLH1/PMS1 complex Sources: GOC:vk